{
  "gene_symbol": "RPL8",
  "term_label": "cytosolic large ribosomal subunit",
  "gene_name": "Large ribosomal subunit protein uL2",
  "gene": "UniProtKB:P62917",
  "term_id": "GO:0022625"
}